Swr1 complex [GO:0000812] (cellular component) Definition: A multisubunit protein complex that is involved in chromatin remodeling. It is required for the incorporation of the histone variant H2AZ into chromatin. In S. cerevisiae, the complex contains Swr1p, a Swi2/Snf2-related ATPase, and 12 additional subunits. Relationships: is_a histone deacetylase complex [GO:0000118]; is a type of GO:0097346; is part of GO:0000228 Also known as: SWR-C References: PMID:14645854, PMID:14690608, PMID:19355820 Sources: GOC:rb